{
  "gene": "UniProtKB:Q7Z4I7",
  "gene_name": "LIM and senescent cell antigen-like-containing domain protein 2",
  "term_label": "Unknown molecular function",
  "gene_symbol": "LIMS2",
  "term_id": "UNKNOWN:0001"
}